{
  "term_label": "regulation of alternative mRNA splicing, via spliceosome",
  "gene_name": "KH domain-containing, RNA-binding, signal transduction-associated protein 1",
  "term_id": "GO:0000381",
  "gene": "UniProtKB:Q07666",
  "gene_symbol": "KHDRBS1"
}